pre-replicative complex assembly involved in bacterial-type DNA replication [GO:0036390] (biological process) Definition: The aggregation, arrangement and bonding together of a set of components to form the bacterial pre-replicative complex, a protein-DNA complex that forms at the bacterial oriC during the initial step of DNA replication and allows the origin to become competent, or 'licensed', for replication. References: PMID:19833870, PMID:21035377, PMID:21895796 Sources: GOC:bf, GOC:bhm, GOC:jh2 Also known as: bacterial pre-RC assembly, bacterial pre-replicative complex assembly Relationships: is a type of GO:1902299; BFO_0000050 bacterial-type DNA replication [GO:0044787]